{
  "gene_symbol": "NR3C2",
  "gene": "UniProtKB:P08235",
  "gene_name": "Mineralocorticoid receptor",
  "term_label": "estrogen response element binding",
  "term_id": "GO:0034056"
}